{
  "gene": "UniProtKB:O14924",
  "gene_symbol": "RGS12",
  "gene_name": "Regulator of G-protein signaling 12",
  "term_label": "cytoplasm",
  "term_id": "GO:0005737"
}